{
  "term_label": "DNA-binding transcription repressor activity, RNA polymerase II-specific",
  "term_id": "GO:0001227",
  "gene_symbol": "KRBOX5",
  "gene_name": "KRAB domain-containing protein 5",
  "gene": "UniProtKB:Q7Z2F6"
}